{
  "gene_symbol": "PAK4",
  "term_label": "protein serine/threonine kinase activity",
  "term_id": "GO:0004674",
  "gene": "UniProtKB:O96013",
  "gene_name": "Serine_threonine-protein kinase PAK 4"
}